protein localization to chromosome, telomeric region [GO:0070198] (biological process) Definition: Any process in which a protein is transported to, or maintained at, the telomeric region of a chromosome. Regulation: regulated by regulation of protein localization to chromosome, telomeric region [GO:1904814]; negatively regulated by negative regulation of protein localization to chromosome, telomeric region [GO:1904815]; positively regulated by GO:1904816 Sources: GOC:BHF, GOC:mah Relationships: is a type of protein localization to chromosome [GO:0034502] Subtypes: protein localization to subtelomeric heterochromatin [GO:1903213] Also known as: protein localisation to chromosome, telomeric region, protein localization to telomere